secondary cell septum [GO:0051077] (cellular component) Definition: Cell wall structures composed of linear polysaccharides which are deposited at both sides of the primary septum at 90 degrees to the primary septum. References: PMID:15194814 Sources: GOC:mtg_sensu Also known as: secondary septum Relationships: is_a division septum [GO:0000935]